{
  "gene_name": "Serine_threonine-protein phosphatase 2A activator",
  "gene_symbol": "PTPA",
  "term_id": "GO:0000159",
  "term_label": "protein phosphatase type 2A complex",
  "gene": "UniProtKB:Q15257"
}